{
  "gene_name": "Beta-soluble NSF attachment protein",
  "term_label": "synaptic transmission, glutamatergic",
  "gene_symbol": "NAPB",
  "term_id": "GO:0035249",
  "gene": "UniProtKB:Q9H115"
}